{
  "gene_name": "Cysteine_serine-rich nuclear protein 3",
  "term_id": "GO:0005634",
  "term_label": "nucleus",
  "gene": "UniProtKB:Q8WYN3",
  "gene_symbol": "CSRNP3"
}